{
  "gene_symbol": "ADD3",
  "term_label": "plasma membrane",
  "term_id": "GO:0005886",
  "gene": "UniProtKB:Q9UEY8",
  "gene_name": "Gamma-adducin"
}